{
  "gene_symbol": "FSD1L",
  "gene": "UniProtKB:Q9BXM9",
  "gene_name": "FSD1-like protein",
  "term_id": "UNKNOWN:0002",
  "term_label": "Unknown biological process"
}